{
  "gene": "UniProtKB:Q8WZB0",
  "term_id": "UNKNOWN:0003",
  "term_label": "Unknown cellular component",
  "gene_name": "Putative uncharacterized protein ERCC6L2-AS1",
  "gene_symbol": "ERCC6L2-AS1"
}